{
  "term_id": "UNKNOWN:0002",
  "gene_symbol": "ZFAND5",
  "term_label": "Unknown biological process",
  "gene": "UniProtKB:O76080",
  "gene_name": "AN1-type zinc finger protein 5"
}